{
  "term_id": "UNKNOWN:0002",
  "gene_symbol": "NUP210",
  "term_label": "Unknown biological process",
  "gene": "UniProtKB:Q8TEM1",
  "gene_name": "Nuclear pore membrane glycoprotein 210"
}